{
  "gene_name": "Septin-11",
  "gene": "UniProtKB:Q9NVA2",
  "term_label": "molecular adaptor activity",
  "gene_symbol": "SEPTIN11",
  "term_id": "GO:0060090"
}